{
  "term_id": "GO:0005886",
  "gene_symbol": "OR7A2P",
  "term_label": "plasma membrane",
  "gene_name": "Putative olfactory receptor 7A2",
  "gene": "UniProtKB:Q8NGA2"
}